cytoplasmic viral factory [GO:0039714] (cellular component) Relationships: is a type of GO:0033655; is_a viral factory [GO:0039713] Subtypes: GO:0039716, GO:0039717, GO:0039718, tube viral factory [GO:0039719], host cell viral assembly compartment [GO:0072517] Definition: A viral factory located in the cytoplasm of a host cell. Sources: VZ:1951